positive regulation of T cell mediated immunity [GO:0002711] (biological process) Subtypes: positive regulation of type IV hypersensitivity [GO:0001809], positive regulation of T cell mediated cytotoxicity [GO:0001916], positive regulation of T cell antigen processing and presentation [GO:0002627], positive regulation of T cell cytokine production [GO:0002726], positive regulation of T cell mediated immune response to tumor cell [GO:0002842], GO:0002851, GO:0035398 Relationships: is a type of positive regulation of lymphocyte mediated immunity [GO:0002708]; is_a regulation of T cell mediated immunity [GO:0002709]; is a type of positive regulation of adaptive immune response based on somatic recombination of immune receptors built from immunoglobulin superfamily domains [GO:0002824]; positively regulates T cell mediated immunity [GO:0002456] Definition: Any process that activates or increases the frequency, rate, or extent of T cell mediated immunity. Also known as: positive regulation of T lymphocyte mediated immunity, positive regulation of T-cell mediated immunity, positive regulation of T-lymphocyte mediated immunity, up regulation of T cell mediated immunity, up-regulation of T cell mediated immunity, upregulation of T cell mediated immunity, activation of T cell mediated immunity, stimulation of T cell mediated immunity Sources: GOC:add